{
  "gene": "UniProtKB:Q9Y613",
  "gene_name": "FH1_FH2 domain-containing protein 1",
  "gene_symbol": "FHOD1",
  "term_id": "GO:0007015",
  "term_label": "actin filament organization"
}